positive regulation of blood coagulation, extrinsic pathway [GO:2000265] (biological process) Sources: GOC:mah Definition: Any process that activates or increases the frequency, rate or extent of blood coagulation, extrinsic pathway. Relationships: is a type of GO:0030194; is a type of GO:2000259; is a type of regulation of blood coagulation, extrinsic pathway [GO:2000263]; positively regulates GO:0007598